{
  "gene": "UniProtKB:Q8NEB7",
  "term_id": "UNKNOWN:0001",
  "gene_symbol": "ACRBP",
  "gene_name": "Acrosin-binding protein",
  "term_label": "Unknown molecular function"
}